{
  "term_id": "GO:0071786",
  "term_label": "endoplasmic reticulum tubular network organization",
  "gene_symbol": "TMEM33",
  "gene_name": "Transmembrane protein 33",
  "gene": "UniProtKB:P57088"
}